protein histidine kinase complex [GO:0009365] (cellular component) Sources: GOC:mah Relationships: is a type of protein kinase complex [GO:1902911] Definition: A complex that possesses protein histidine kinase activity.